{
  "term_label": "Unknown molecular function",
  "term_id": "UNKNOWN:0001",
  "gene": "UniProtKB:Q6ZSR9",
  "gene_name": "Uncharacterized protein FLJ45252",
  "gene_symbol": "Q6ZSR9"
}